{
  "gene": "UniProtKB:Q07812",
  "gene_name": "Apoptosis regulator BAX",
  "gene_symbol": "BAX",
  "term_label": "extrinsic apoptotic signaling pathway in absence of ligand",
  "term_id": "GO:0097192"
}